regulation of vascular endothelial growth factor production [GO:0010574] (biological process) Definition: Any process that modulates the frequency, rate, or extent of production of vascular endothelial growth factor. Sources: GOC:rl Relationships: is a type of regulation of cytokine production [GO:0001817]; regulates GO:0010573 Subtypes: positive regulation of vascular endothelial growth factor production [GO:0010575], negative regulation of vascular endothelial growth factor production [GO:1904046]